spongiotrophoblast cell proliferation [GO:0060720] (biological process) Relationships: is a type of cell proliferation involved in embryonic placenta development [GO:0060722]; is part of spongiotrophoblast layer developmental growth [GO:0090214] Definition: The multiplication or reproduction of spongiotrophoblast cells, resulting in the expansion of the population in the spongiotrophoblast layer. Regulation: RO_0002211 by regulation of spongiotrophoblast cell proliferation [GO:0060721] Sources: GOC:dph